{
  "gene": "UniProtKB:A8MUU9",
  "gene_name": "Putative uncharacterized protein ENSP00000383309",
  "term_id": "UNKNOWN:0002",
  "gene_symbol": "A8MUU9",
  "term_label": "Unknown biological process"
}